regulation of myofibroblast differentiation [GO:1904760] (biological process) Definition: Any process that modulates the frequency, rate or extent of myofibroblast differentiation. References: PMID:20533548 Sources: GOC:BHF, GOC:BHF_miRNA, GOC:TermGenie, GOC:rph, GO_REF:0000058 Also known as: regulation of myofibroblast cell differentiation Relationships: is a type of regulation of cell differentiation [GO:0045595]; regulates GO:0036446 Subtypes: negative regulation of myofibroblast differentiation [GO:1904761], positive regulation of myofibroblast differentiation [GO:1904762]